{
  "gene_symbol": "RAB8A",
  "gene": "UniProtKB:P61006",
  "term_label": "neurotransmitter receptor transport to postsynaptic membrane",
  "term_id": "GO:0098969",
  "gene_name": "Ras-related protein Rab-8A"
}